{
  "gene_symbol": "MYNN",
  "term_label": "Unknown cellular component",
  "gene_name": "Myoneurin",
  "term_id": "UNKNOWN:0003",
  "gene": "UniProtKB:Q9NPC7"
}